quercetin 3-O-glucosyltransferase activity [GO:0080043] (molecular function) Definition: Catalysis of the transfer of a glucosyl group from UDP-glucose to the 3-hydroxy group of a quercetin molecule. Relationships: is a type of UDP-glucosyltransferase activity [GO:0035251] References: PMID:15352060